{
  "term_label": "nucleus",
  "gene_symbol": "ZNHIT6",
  "gene": "UniProtKB:Q9NWK9",
  "gene_name": "Box C_D snoRNA protein 1",
  "term_id": "GO:0005634"
}